{
  "gene_name": "Cilium assembly protein DZIP1",
  "term_id": "GO:0060271",
  "term_label": "cilium assembly",
  "gene": "UniProtKB:Q86YF9",
  "gene_symbol": "DZIP1"
}